pinene synthase activity [GO:0050550] (molecular function) Definition: Catalysis of the reaction: geranyl diphosphate = pinene + diphosphate. This reaction can produce (1R,5R)-alpha-pinene, (1S,5S)-alpha-pinene, (1R,5R)-beta-pinene and (1S,5S)-beta-pinene. References: PMID:21385377, PMID:23679205 Also known as: (-)-(1S,5S)-pinene synthase activity, alpha-pinene synthase activity, beta-pinene synthase activity, beta-geraniolene synthase activity Relationships: is a type of terpene synthase activity [GO:0010333]